{
  "gene": "UniProtKB:Q8WW12",
  "gene_name": "PEST proteolytic signal-containing nuclear protein",
  "term_label": "nucleus",
  "gene_symbol": "PCNP",
  "term_id": "GO:0005634"
}